chromatin-nuclear membrane anchor activity [GO:0140707] (molecular function) References: PMID:24184107, PMID:31048766 Subtypes: heterochromatin-nuclear membrane anchor activity [GO:0062239], euchromatin-nuclear membrane anchor activity [GO:0062240] Relationships: is a type of protein-membrane adaptor activity [GO:0043495] Definition: Binding to chromatin and the nuclear inner membrane, in order to establish and maintain the heterochromatin location and organization, or to enable equal segregation of the nuclear membrane during mitosis.